{
  "gene": "UniProtKB:P01112",
  "term_id": "GO:0005886",
  "gene_symbol": "HRAS",
  "term_label": "plasma membrane",
  "gene_name": "GTPase HRas"
}